{
  "gene_symbol": "WIPI1",
  "term_label": "glycophagy",
  "gene_name": "WD repeat domain phosphoinositide-interacting protein 1",
  "term_id": "GO:0061723",
  "gene": "UniProtKB:Q5MNZ9"
}